{
  "gene_symbol": "OTOP1",
  "term_id": "GO:0042802",
  "gene_name": "Proton channel OTOP1",
  "gene": "UniProtKB:Q7RTM1",
  "term_label": "identical protein binding"
}